tubulin-tyrosine ligase activity [GO:0004835] (molecular function) Definition: Catalysis of the reaction: ATP + detyrosinated alpha-tubulin + L-tyrosine = alpha-tubulin + ADP + phosphate. Sources: EC:6.3.2.25 Also known as: tubulinyl-tyrosine ligase activity, TTL activity, alpha-tubulin:L-tyrosine ligase (ADP-forming) Relationships: is a type of acid-amino acid ligase activity [GO:0016881]; is a type of catalytic activity, acting on a protein [GO:0140096]